{
  "gene": "UniProtKB:Q6V1P9",
  "term_label": "epithelial cell differentiation",
  "gene_name": "Protocadherin-23",
  "gene_symbol": "DCHS2",
  "term_id": "GO:0030855"
}